{
  "gene": "UniProtKB:Q9Y592",
  "term_label": "Unknown molecular function",
  "gene_symbol": "CEP83",
  "term_id": "UNKNOWN:0001",
  "gene_name": "Centrosomal protein of 83 kDa"
}